{
  "gene_symbol": "SLC11A2",
  "gene_name": "Natural resistance-associated macrophage protein 2",
  "term_label": "iron ion transmembrane transport",
  "gene": "UniProtKB:P49281",
  "term_id": "GO:0034755"
}